{
  "gene_name": "Tubulin-folding cofactor B",
  "gene_symbol": "TBCB",
  "gene": "UniProtKB:Q99426",
  "term_label": "microtubule plus-end",
  "term_id": "GO:0035371"
}